{
  "gene": "UniProtKB:O75093",
  "gene_name": "Slit homolog 1 protein",
  "term_label": "Roundabout binding",
  "term_id": "GO:0048495",
  "gene_symbol": "SLIT1"
}